{
  "gene_symbol": "XNDC1N",
  "term_label": "Unknown molecular function",
  "gene": "UniProtKB:Q6ZNB5",
  "gene_name": "Protein XNDC1N",
  "term_id": "UNKNOWN:0001"
}